positive regulation of TOR signaling [GO:0032008] (biological process) Sources: GOC:mah Also known as: positive regulation of TOR signaling pathway, positive regulation of TOR signalling pathway, positive regulation of target of rapamycin signaling pathway, positive regulation of target of rapamycin signalling pathway, up regulation of TOR signaling pathway, up-regulation of TOR signaling pathway, upregulation of TOR signaling pathway, activation of TOR signaling pathway, stimulation of TOR signaling pathway, positive regulation of TOR signaling cascade Relationships: is a type of GO:0032006; is a type of positive regulation of intracellular signal transduction [GO:1902533]; positively regulates GO:0031929 Subtypes: GO:1904263, positive regulation of TORC2 signaling [GO:1904515] Definition: Any process that activates or increases the frequency, rate or extent of TOR signaling.